{
  "gene_symbol": "NME2P1",
  "gene_name": "Putative nucleoside diphosphate kinase",
  "gene": "UniProtKB:O60361",
  "term_label": "nucleoside diphosphate kinase activity",
  "term_id": "GO:0004550"
}